{
  "gene": "UniProtKB:P26439",
  "term_id": "GO:0006694",
  "gene_name": "3 beta-hydroxysteroid dehydrogenase_Delta 5--4-isomerase type 2",
  "gene_symbol": "HSD3B2",
  "term_label": "steroid biosynthetic process"
}